{
  "gene_name": "Protein HEATR9",
  "term_label": "Unknown molecular function",
  "gene_symbol": "HEATR9",
  "gene": "UniProtKB:A2RTY3",
  "term_id": "UNKNOWN:0001"
}